{
  "term_label": "phosphatidylethanolamine binding",
  "gene_symbol": "GABARAPL3",
  "term_id": "GO:0008429",
  "gene_name": "Gamma-aminobutyric acid receptor-associated protein-like 3",
  "gene": "UniProtKB:Q9BY60"
}